cell proliferation involved in endocardial cushion morphogenesis [GO:1905315] (biological process) References: PMID:20652948 Sources: GOC:BHF, GOC:TermGenie, GOC:rl, GO_REF:0000060 Definition: Any cell proliferation that is involved in endocardial cushion morphogenesis. Relationships: is_a GO:0061323; is part of endocardial cushion morphogenesis [GO:0003203]